protein-phosphocysteine-N,N'-diacetylchitobiose phosphotransferase system transporter activity [GO:0090566] (molecular function) References: PMID:10913119 Sources: GOC:am Relationships: is a type of protein-phosphocysteine-sugar phosphotransferase activity [GO:0090563] Definition: Catalysis of the PEP-dependent, phosphoryl transfer-driven transport of substances across a membrane. The transport happens by catalysis of the reaction: protein S-phosphocysteine + N,N'-diacetylchitobiose(out) = protein cysteine + N,N'-diacetylchitobiose phosphate(in).